tRNA (uridine) methyltransferase activity [GO:0016300] (MF) Sources: GOC:mah Subtypes: tRNA (5-methylaminomethyl-2-thiouridylate)(34)-methyltransferase activity [GO:0004808], GO:0030697, tRNA (uracil(54)-C5)-methyltransferase activity, 5,10-methylenetetrahydrofolate-dependent [GO:0047151], tRNA (5-carboxymethoxyuridine(34)-5-O)-methyltransferase activity [GO:0097697], GO:0106335, GO:0141101, tRNA (5-carboxymethylaminomethyluridine(34)-2'-O)-methyltransferase activity [GO:0141102], tRNA (cytidine(32)/uridine(32)-2'-O)-methyltransferase activity [GO:0160206] Also known as: tRNA (uracil) methyltransferase activity Relationships: is a type of GO:0008175 Definition: Catalysis of the transfer of a methyl group from a donor to a uracil residue in a tRNA molecule.